{
  "gene_name": "Protein bicaudal D homolog 1",
  "gene_symbol": "BICD1",
  "term_id": "GO:0048260",
  "term_label": "positive regulation of receptor-mediated endocytosis",
  "gene": "UniProtKB:Q96G01"
}